{
  "gene_symbol": "PPP3CA",
  "term_id": "GO:0005737",
  "gene_name": "Protein phosphatase 3 catalytic subunit alpha",
  "term_label": "cytoplasm",
  "gene": "UniProtKB:Q08209"
}